choline transport [GO:0015871] (biological process) Sources: GOC:ai Definition: The directed movement of choline into, out of or within a cell, or between cells, by means of some agent such as a transporter or pore. Choline (2-hydroxyethyltrimethylammonium) is an amino alcohol that occurs widely in living organisms as a constituent of certain types of phospholipids and in the neurotransmitter acetylcholine. Relationships: is a type of GO:0015695; is a type of nitrogen compound transport [GO:0071705]